{
  "term_label": "microtubule minus-end binding",
  "gene": "UniProtKB:Q96RT8",
  "term_id": "GO:0051011",
  "gene_name": "Gamma-tubulin complex component 5",
  "gene_symbol": "TUBGCP5"
}